{
  "term_label": "animal organ development",
  "gene_name": "Pro-neuregulin-3, membrane-bound isoform",
  "gene_symbol": "NRG3",
  "term_id": "GO:0048513",
  "gene": "UniProtKB:P56975"
}